{
  "term_label": "formation of translation preinitiation complex",
  "gene_name": "Eukaryotic translation initiation factor 2 subunit 2",
  "term_id": "GO:0001731",
  "gene": "UniProtKB:P20042",
  "gene_symbol": "EIF2S2"
}